layer formation in cerebral cortex [GO:0021819] (biological process) References: PMID:12626695 Sources: GOC:cls, GOC:dgh, GOC:dph, GOC:jid, GO_REF:0000021 Also known as: cerebral cortex lamination Relationships: is a type of GO:0048646; is part of GO:0021801 Definition: The detachment of cells from radial glial fibers at the appropriate time when they cease to migrate and form distinct layer in the cerebral cortex.